{
  "term_id": "UNKNOWN:0001",
  "gene": "UniProtKB:Q9HCH0",
  "gene_symbol": "NCKAP5L",
  "gene_name": "Nck-associated protein 5-like",
  "term_label": "Unknown molecular function"
}